{
  "gene_name": "Mitochondrial folate transporter_carrier",
  "gene": "UniProtKB:Q9H2D1",
  "gene_symbol": "SLC25A32",
  "term_id": "GO:0005739",
  "term_label": "mitochondrion"
}